cyanamide metabolic process [GO:0018890] (biological process) Definition: The chemical reactions and pathways involving cyanamide, NCNH2, a cyanide compound which has been used as a fertilizer, defoliant and in many manufacturing processes. It often occurs as the calcium salt, sometimes also referred to as cyanamide. The citrated calcium salt is used in the treatment of alcoholism. Relationships: is_a xenobiotic metabolic process [GO:0006805]; is a type of nitrile metabolic process [GO:0050898] Also known as: cyanamide metabolism Sources: GOC:curators